{
  "gene": "UniProtKB:P0DX01",
  "gene_name": "Golgin subfamily A member 6-like protein 25",
  "term_id": "UNKNOWN:0003",
  "gene_symbol": "GOLGA6L25",
  "term_label": "Unknown cellular component"
}